{
  "term_label": "Unknown molecular function",
  "term_id": "UNKNOWN:0001",
  "gene": "UniProtKB:Q5F1R6",
  "gene_name": "DnaJ homolog subfamily C member 21",
  "gene_symbol": "DNAJC21"
}